{
  "gene_symbol": "FBXO48",
  "term_label": "cytoplasm",
  "gene_name": "F-box only protein 48",
  "gene": "UniProtKB:Q5FWF7",
  "term_id": "GO:0005737"
}